{
  "term_id": "GO:1990604",
  "gene_name": "Serine_threonine-protein kinase_endoribonuclease IRE1",
  "term_label": "IRE1-TRAF2-ASK1 complex",
  "gene": "UniProtKB:O75460",
  "gene_symbol": "ERN1"
}